{
  "gene_symbol": "DNAJB1",
  "gene_name": "DnaJ homolog subfamily B member 1",
  "gene": "UniProtKB:P25685",
  "term_label": "protein folding",
  "term_id": "GO:0006457"
}